{
  "gene_name": "Collagen alpha-2(IX) chain",
  "gene": "UniProtKB:Q14055",
  "term_id": "GO:0030020",
  "gene_symbol": "COL9A2",
  "term_label": "extracellular matrix structural constituent conferring tensile strength"
}